{
  "gene_name": "Protein PIGBOS1",
  "term_label": "Unknown cellular component",
  "gene": "UniProtKB:A0A0B4J2F0",
  "gene_symbol": "PIGBOS1",
  "term_id": "UNKNOWN:0003"
}